{
  "term_label": "nucleus",
  "gene_symbol": "ZBTB46",
  "gene_name": "Zinc finger and BTB domain-containing protein 46",
  "gene": "UniProtKB:Q86UZ6",
  "term_id": "GO:0005634"
}